{
  "term_label": "tubulin binding",
  "gene_name": "Tubulin polyglutamylase TTLL7",
  "gene": "UniProtKB:Q6ZT98",
  "gene_symbol": "TTLL7",
  "term_id": "GO:0015631"
}